tight junction assembly [GO:0120192] (biological process) Relationships: is a type of GO:0007043; is a type of tight junction organization [GO:0120193] Sources: GOC:rl Definition: A cellular process that results in the aggregation, arrangement and bonding together of a set of components to form a tight junction. A tight junction seals cells together in an epithelium in a way that prevents even small molecules from leaking from one side of the sheet to the other. Subtypes: septate junction assembly [GO:0019991], bicellular tight junction assembly [GO:0070830], GO:1904274 Also known as: occluding cell junction assembly, occluding junction assembly